{
  "gene": "UniProtKB:P0DUQ1",
  "term_id": "GO:0031462",
  "term_label": "Cul2-RING ubiquitin ligase complex",
  "gene_symbol": "PRAMEF15",
  "gene_name": "PRAME family member 15"
}